{
  "gene_symbol": "TJP1",
  "term_id": "GO:0005886",
  "gene": "UniProtKB:Q07157",
  "term_label": "plasma membrane",
  "gene_name": "Tight junction protein ZO-1"
}